{
  "term_label": "respiratory chain complex I",
  "gene_name": "NADH-ubiquinone oxidoreductase chain 3",
  "gene_symbol": "MT-ND3",
  "gene": "UniProtKB:P03897",
  "term_id": "GO:0045271"
}